{
  "gene": "UniProtKB:Q9UJM8",
  "term_label": "Unknown biological process",
  "gene_symbol": "HAO1",
  "term_id": "UNKNOWN:0002",
  "gene_name": "2-Hydroxyacid oxidase 1"
}